site-specific DNA replication termination at RTS1 barrier [GO:0071171] (biological process) References: PMID:12009298, PMID:18723894 Sources: GOC:vw Definition: A DNA replication termination process that takes place at the RTS1 termination site in the mating type locus, in a specific direction required for subsequent imprinting and mating-type switching. Relationships: is a type of site-specific DNA replication termination [GO:0071170]; is part of mating-type locus imprinting [GO:0071515]